{
  "gene_name": "tRNA 2'-phosphotransferase 1",
  "term_id": "UNKNOWN:0003",
  "gene_symbol": "TRPT1",
  "gene": "UniProtKB:Q86TN4",
  "term_label": "Unknown cellular component"
}